{
  "gene": "UniProtKB:Q6UXR6",
  "term_id": "UNKNOWN:0003",
  "gene_symbol": "UNQ6494_PRO21346",
  "term_label": "Unknown cellular component",
  "gene_name": "Putative uncharacterized protein UNQ6494_PRO21346"
}